leukocyte aggregation [GO:0070486] (biological process) References: PMID:12972508 Sources: GOC:sl Also known as: immune cell aggregation, leucocyte aggregation, white blood cell aggregation, white corpuscle aggregation Subtypes: monocyte aggregation [GO:0070487], GO:0070488, GO:0071593 Definition: The adhesion of one leukocyte to one or more other leukocytes via adhesion molecules. Relationships: is a type of leukocyte cell-cell adhesion [GO:0007159]